{
  "term_id": "UNKNOWN:0001",
  "gene_symbol": "C11orf96",
  "term_label": "Unknown molecular function",
  "gene_name": "Uncharacterized protein C11orf96",
  "gene": "UniProtKB:Q7Z7L8"
}